oxoglutarate:malate antiporter activity [GO:0015367] (molecular function) Definition: Enables the transfer of a solute or solutes from one side of a membrane to the other according to the reaction: oxoglutarate(out) + malate(in) = oxoglutarate(in) + malate(out). Sources: TC:2.A.29.2.1 Also known as: 2-oxoglutarate/malate carrier protein Relationships: is a type of alpha-ketoglutarate transmembrane transporter activity [GO:0015139]; is a type of malate transmembrane transporter activity [GO:0015140]; is a type of GO:0015297